{
  "term_label": "Unknown cellular component",
  "gene_symbol": "SSR2",
  "gene": "UniProtKB:P43308",
  "gene_name": "Translocon-associated protein subunit beta",
  "term_id": "UNKNOWN:0003"
}